regulation of SNARE complex assembly [GO:0035542] (biological process) Definition: Any process that modulates the frequency, rate or extent of assembly of the SNARE complex. The SNARE complex is a protein complex involved in membrane fusion; a stable ternary complex consisting of a four-helix bundle, usually formed from one R-SNARE and three Q-SNAREs with an ionic layer sandwiched between hydrophobic layers. Sources: GOC:rb Relationships: is a type of regulation of protein-containing complex assembly [GO:0043254]; RO_0002211 GO:0035493 Subtypes: positive regulation of SNARE complex assembly [GO:0035543], negative regulation of SNARE complex assembly [GO:0035544]